{
  "term_label": "Unknown molecular function",
  "gene_name": "THAP domain-containing protein 2",
  "gene": "UniProtKB:Q9H0W7",
  "gene_symbol": "THAP2",
  "term_id": "UNKNOWN:0001"
}